{
  "gene_symbol": "CYP11B1",
  "term_id": "GO:0034650",
  "gene": "UniProtKB:P15538",
  "term_label": "cortisol metabolic process",
  "gene_name": "Cytochrome P450 11B1, mitochondrial"
}